{
  "gene_name": "Putative G-protein coupled receptor GPR32P1",
  "gene_symbol": "GPR32P1",
  "term_label": "complement receptor activity",
  "term_id": "GO:0004875",
  "gene": "UniProtKB:Q8NGA4"
}